{
  "term_id": "GO:0000122",
  "gene_name": "Zinc finger protein 814",
  "gene_symbol": "ZNF814",
  "gene": "UniProtKB:B7Z6K7",
  "term_label": "negative regulation of transcription by RNA polymerase II"
}